{
  "term_label": "nucleus",
  "gene_symbol": "L3MBTL2",
  "gene_name": "Lethal(3)malignant brain tumor-like protein 2",
  "term_id": "GO:0005634",
  "gene": "UniProtKB:Q969R5"
}